adipokinetic hormone receptor binding [GO:0097005] (molecular function) Relationships: is a type of peptide hormone receptor binding [GO:0051428] References: PMID:11904407 Sources: GOC:sart Also known as: AKH receptor binding Definition: Binding to an adipokinetic hormone receptor. Adipokinetic hormones (AKHs) are peptide hormones that are involved in the mobilization of sugar and lipids from the insect fat body during energy-requiring activities such as flight and locomotion. They also contribute to hemolymph sugar homeostasis.